{
  "term_id": "GO:0005579",
  "gene_symbol": "C7",
  "gene_name": "Complement component C7",
  "term_label": "membrane attack complex",
  "gene": "UniProtKB:P10643"
}